{
  "gene_name": "Forkhead box protein J3",
  "term_label": "regulation of transcription by RNA polymerase II",
  "gene": "UniProtKB:Q9UPW0",
  "gene_symbol": "FOXJ3",
  "term_id": "GO:0006357"
}